regulation of cyanophore differentiation [GO:0048781] (biological process) Definition: Any process that modulates the frequency, rate or extent of cyanophore differentiation. Sources: GOC:mh Relationships: is a type of regulation of pigment cell differentiation [GO:0050932]; regulates cyanophore differentiation [GO:0048774] Subtypes: negative regulation of cyanophore differentiation [GO:0048782], positive regulation of cyanophore differentiation [GO:0048783]